{
  "gene": "UniProtKB:Q9UEU0",
  "gene_symbol": "VTI1B",
  "term_label": "ER to Golgi transport vesicle membrane",
  "gene_name": "Vesicle transport through interaction with t-SNAREs homolog 1B",
  "term_id": "GO:0012507"
}